{
  "gene": "UniProtKB:Q9NZH0",
  "gene_name": "G-protein coupled receptor family C group 5 member B",
  "term_id": "GO:0005886",
  "gene_symbol": "GPRC5B",
  "term_label": "plasma membrane"
}